lithium:proton antiporter activity [GO:0010348] (molecular function) Relationships: is a type of metal cation:proton antiporter activity [GO:0051139] Definition: Enables the transfer of a solute or solutes from one side of a membrane to the other according to the reaction: Li+(in) + H+(out) = Li+(out) + H+(in). References: PMID:17270011 Also known as: lithium:hydrogen antiporter activity